{
  "term_label": "nucleus",
  "gene": "UniProtKB:Q9HAH1",
  "term_id": "GO:0005634",
  "gene_name": "Zinc finger protein 556",
  "gene_symbol": "ZNF556"
}